berbamunine biosynthetic process [GO:0035833] (biological process) Sources: GOC:yaf Definition: The chemical reactions and pathways resulting in the formation of berbamunine, an isoquinoline alkaloid. Also known as: berbamunine anabolism, berbamunine biosynthesis, berbamunine formation, berbamunine synthesis Relationships: is a type of benzyl isoquinoline alkaloid biosynthetic process [GO:0009708]